{
  "gene": "UniProtKB:P0DPK5",
  "term_label": "nucleosomal DNA binding",
  "term_id": "GO:0031492",
  "gene_name": "Histone H3.X",
  "gene_symbol": "H3Y2"
}